{
  "gene_name": "T cell receptor beta variable 13",
  "gene": "UniProtKB:A0A0A6YYD4",
  "gene_symbol": "TRBV13",
  "term_label": "cell surface receptor signaling pathway",
  "term_id": "GO:0007166"
}